{
  "gene_name": "[Pyruvate dehydrogenase (acetyl-transferring)] kinase isozyme 1, mitochondrial",
  "gene_symbol": "PDK1",
  "term_label": "regulation of glucose metabolic process",
  "gene": "UniProtKB:Q15118",
  "term_id": "GO:0010906"
}